{
  "term_label": "ATPase-coupled intramembrane lipid transporter activity",
  "gene_name": "Probable phospholipid-transporting ATPase IIA",
  "gene_symbol": "ATP9A",
  "gene": "UniProtKB:O75110",
  "term_id": "GO:0140326"
}